granulocyte colony-stimulating factor receptor binding [GO:0005130] (molecular function) Sources: GOC:ai Relationships: is a type of GO:0005126; is a type of growth factor receptor binding [GO:0070851] Definition: Binding to a granulocyte colony-stimulating factor receptor. Also known as: G-CSF receptor ligand, GC-SF receptor ligand, granulocyte colony stimulating factor receptor binding, granulocyte colony-stimulating factor, granulocyte colony-stimulating factor receptor ligand